{
  "gene": "UniProtKB:Q9NZQ8",
  "gene_name": "Transient receptor potential cation channel subfamily M member 5",
  "gene_symbol": "TRPM5",
  "term_id": "GO:0005227",
  "term_label": "calcium-activated cation channel activity"
}